{
  "gene_symbol": "MCTP1",
  "gene": "UniProtKB:Q6DN14",
  "term_id": "GO:0005509",
  "term_label": "calcium ion binding",
  "gene_name": "Multiple C2 and transmembrane domain-containing protein 1"
}